{
  "term_id": "GO:0000981",
  "gene": "UniProtKB:Q96GE5",
  "term_label": "DNA-binding transcription factor activity, RNA polymerase II-specific",
  "gene_symbol": "ZNF799",
  "gene_name": "Zinc finger protein 799"
}